{
  "term_label": "Golgi apparatus",
  "gene_symbol": "CLCN5",
  "term_id": "GO:0005794",
  "gene_name": "H(+)_Cl(-) exchange transporter 5",
  "gene": "UniProtKB:P51795"
}